negative regulation of pancreatic juice secretion [GO:0090188] (biological process) Definition: Any process that decreases the rate, frequency or extent of pancreatic juice secretion, the regulated release of pancreatic juice by the exocrine pancreas into the upper part of the intestine. Sources: GOC:BHF, GOC:dph, GOC:tb Relationships: is a type of GO:0051048; is a type of negative regulation of digestive system process [GO:0060457]; is a type of GO:0090186; negatively regulates pancreatic juice secretion [GO:0030157]